tri-n-butyltin metabolic process [GO:0018944] (biological process) Relationships: is a type of organometal metabolic process [GO:0018942] Definition: The chemical reactions and pathways involving tri-n-butyltin, an organometallic compound composed of three butyl chains attached to a tin atom. Tri-n-butyltin is used as an antifouling agent in ship bottom paints and can be toxic to many marine organisms. Also known as: tri-n-butyltin metabolism Sources: GOC:ai, UM-BBD_pathwayID:tbt